stem cell division [GO:0017145] (biological process) Regulation: regulated by regulation of stem cell division [GO:2000035] Definition: The self-renewing division of a stem cell. A stem cell is an undifferentiated cell, in the embryo or adult, that can undergo unlimited division and give rise to one or several different cell types. Subtypes: GO:0042078, GO:0048103, asymmetric stem cell division [GO:0098722], GO:0098724 Relationships: is_a GO:0051301 Also known as: stem cell renewal Sources: GOC:jid, ISBN:0582227089